{
  "term_id": "GO:0034432",
  "gene": "UniProtKB:Q96G61",
  "gene_symbol": "NUDT11",
  "gene_name": "Diphosphoinositol polyphosphate phosphohydrolase 3-beta",
  "term_label": "bis(5'-adenosyl)-pentaphosphatase activity"
}